{
  "gene": "UniProtKB:Q8NHX9",
  "term_id": "GO:0019722",
  "gene_symbol": "TPCN2",
  "gene_name": "Two pore channel protein 2",
  "term_label": "calcium-mediated signaling"
}